{
  "term_id": "GO:0000976",
  "term_label": "transcription cis-regulatory region binding",
  "gene_symbol": "ZNF629",
  "gene": "UniProtKB:Q9UEG4",
  "gene_name": "Zinc finger protein 629"
}